{
  "gene_symbol": "BANK1",
  "gene_name": "B-cell scaffold protein with ankyrin repeats",
  "gene": "UniProtKB:Q8NDB2",
  "term_label": "Unknown cellular component",
  "term_id": "UNKNOWN:0003"
}